adenylylsulfate kinase activity [GO:0004020] (molecular function) Sources: EC:2.7.1.25 Definition: Catalysis of the reaction: adenosine 5'-phosphosulfate + ATP = 3'-phosphoadenylyl sulfate + ADP + H+. Relationships: is a type of kinase activity [GO:0016301]; is a type of GO:0016773 Also known as: adenosine-5'-phosphosulfate 3'-phosphotransferase activity, adenosine-5'-phosphosulphate 3'-phosphotransferase activity, adenylyl-sulfate kinase activity, adenylyl-sulphate kinase activity, 5'-phosphoadenosine sulfate kinase activity, APS kinase activity, ATP:adenylyl-sulfate 3'-phosphotransferase activity, adenosine 5'-phosphosulfate kinase activity, adenosine phosphosulfate kinase activity, adenosine phosphosulfokinase activity, adenosine-5'-phosphosulfate-3'-phosphokinase activity, adenylylsulfate kinase (phosphorylating)